{
  "term_id": "GO:0043328",
  "gene_symbol": "PTPN23",
  "gene_name": "Tyrosine-protein phosphatase non-receptor type 23",
  "term_label": "protein transport to vacuole involved in ubiquitin-dependent protein catabolic process via the multivesicular body sorting pathway",
  "gene": "UniProtKB:Q9H3S7"
}